{
  "gene_symbol": "UPK1A",
  "gene_name": "Uroplakin-1a",
  "term_id": "UNKNOWN:0001",
  "gene": "UniProtKB:O00322",
  "term_label": "Unknown molecular function"
}